{
  "term_label": "negative regulation of interleukin-1 beta production",
  "gene_name": "Leukocyte elastase inhibitor",
  "term_id": "GO:0032691",
  "gene": "UniProtKB:P30740",
  "gene_symbol": "SERPINB1"
}